{
  "gene_symbol": "B4GAT1",
  "gene_name": "Beta-1,4-glucuronyltransferase 1",
  "term_label": "Golgi apparatus",
  "gene": "UniProtKB:O43505",
  "term_id": "GO:0005794"
}